{
  "gene_symbol": "RYR3",
  "gene": "UniProtKB:Q15413",
  "term_label": "striated muscle contraction",
  "term_id": "GO:0006941",
  "gene_name": "Ryanodine receptor 3"
}